{
  "gene": "UniProtKB:P43166",
  "gene_symbol": "CA7",
  "term_label": "regulation of intracellular pH",
  "term_id": "GO:0051453",
  "gene_name": "Carbonic anhydrase 7"
}